4-alpha-glucanotransferase activity [GO:0004134] (molecular function) Relationships: is a type of hexosyltransferase activity [GO:0016758] Sources: EC:2.4.1.25 Also known as: 1,4-alpha-D-glucan:1,4-alpha-D-glucan 4-alpha-D-glycosyltransferase activity, D-enzyme activity, amylomaltase activity, debranching enzyme maltodextrin glycosyltransferase activity, dextrin glycosyltransferase activity, dextrin transglycosylase activity, disproportionating enzyme activity, oligo-1,4-1,4-glucantransferase activity Definition: Catalysis of the transfer of a segment of a (1->4)-alpha-D-glucan to a new 4-position in an acceptor, which may be glucose or (1->4)-alpha-D-glucan.